{
  "term_label": "Unknown molecular function",
  "term_id": "UNKNOWN:0001",
  "gene_symbol": "ZFYVE9",
  "gene_name": "Zinc finger FYVE domain-containing protein 9",
  "gene": "UniProtKB:O95405"
}